{
  "gene": "UniProtKB:Q9H223",
  "term_label": "endocytosis",
  "term_id": "GO:0006897",
  "gene_symbol": "EHD4",
  "gene_name": "EH domain-containing protein 4"
}